{
  "term_id": "GO:0035098",
  "gene_name": "Histone-lysine N-methyltransferase EZH1",
  "term_label": "ESC/E(Z) complex",
  "gene_symbol": "EZH1",
  "gene": "UniProtKB:Q92800"
}